methylaspartate mutase activity [GO:0050097] (molecular function) Relationships: is a type of GO:0016866 Also known as: L-threo-3-methylaspartate carboxy-aminomethylmutase activity, b-methylaspartate-glutamate mutase activity, beta-methylaspartate-glutamate mutase activity, glutamate isomerase activity, glutamate mutase activity, glutamic acid isomerase activity, glutamic acid mutase activity, glutamic isomerase activity, glutamic mutase activity, methylaspartic acid mutase activity Sources: EC:5.4.99.1, RHEA:12857 Definition: Catalysis of the reaction: threo-3-methyl-L-aspartate = L-glutamate.